contact guidance [GO:0009990] (biological process) Relationships: is a type of cell-matrix recognition [GO:0009989] Sources: ISBN:0824072820 Definition: Cell recognition involving the deposition of specific pathways in the extracellular matrix that guide migrating cells.